coreceptor-mediated virion attachment to host cell [GO:0046814] (biological process) Also known as: virion attachment, binding of host cell surface coreceptor Relationships: is a type of virion attachment to host cell [GO:0019062]; BFO_0000051 GO:0039706 Definition: The process by which a virion attaches to a host cell by binding to a co-receptor on the host cell surface. Sources: ISBN:0879694971